{
  "term_label": "GDP-mannose 4,6-dehydratase activity",
  "gene_symbol": "GMDS",
  "gene_name": "GDP-mannose 4,6 dehydratase",
  "gene": "UniProtKB:O60547",
  "term_id": "GO:0008446"
}